{
  "term_id": "GO:0005737",
  "term_label": "cytoplasm",
  "gene_symbol": "FGF2",
  "gene_name": "Fibroblast growth factor 2",
  "gene": "UniProtKB:P09038"
}